{
  "term_id": "GO:0006086",
  "gene": "UniProtKB:P10515",
  "gene_name": "Dihydrolipoyllysine-residue acetyltransferase component of pyruvate dehydrogenase complex, mitochondrial",
  "gene_symbol": "DLAT",
  "term_label": "pyruvate decarboxylation to acetyl-CoA"
}